positive regulation of activation of membrane attack complex [GO:0001970] (biological process) Definition: Any process that activates, maintains or increases the frequency, rate or extent of the activation of the membrane attack complex components of the complement cascade. Relationships: is a type of GO:0001969; is a type of positive regulation of complement activation [GO:0045917]; RO_0002213 activation of membrane attack complex [GO:0001905] Sources: GOC:hjd Also known as: positive regulation of MAC assembly, positive regulation of MAC formation, positive regulation of activation of MAC, positive regulation of membrane attack complex assembly, positive regulation of membrane attack complex formation, up regulation of activation of membrane attack complex, up-regulation of activation of membrane attack complex, upregulation of activation of membrane attack complex, activation of activation of membrane attack complex, positive regulation of activation of TCC, positive regulation of activation of terminal complement complex, positive regulation of activation of the terminal complement cascade, stimulation of activation of membrane attack complex